venous blood vessel morphogenesis [GO:0048845] (biological process) Definition: The process in which the anatomical structures of venous blood vessels are generated and organized. Veins are blood vessels that transport blood from the body and its organs to the heart. References: PMID:16740480 Sources: GOC:dsf Also known as: vein morphogenesis, venous morphogenesis Relationships: is_a blood vessel morphogenesis [GO:0048514]; is part of GO:0060841 Subtypes: coronary vein morphogenesis [GO:0003169], GO:0060577, superior vena cava morphogenesis [GO:0060578], GO:0061116